{
  "gene": "UniProtKB:Q96IK5",
  "term_id": "UNKNOWN:0001",
  "gene_name": "Germ cell-less protein-like 1",
  "term_label": "Unknown molecular function",
  "gene_symbol": "GMCL1"
}